Seh1-associated complex [GO:0035859] (cellular component) Definition: A GTPase-activating protein (GAP) complex that regulates TORC1 signaling by interacting with the Rag GTPase. In S. cerevisiae the complex contains Seh1p, Sec13p, Npr2p, Npr3p, Iml1p, Mtc5p, Rtc1p, and Sea4p. Relationships: is_a GO:0032991 Also known as: GATOR complex, SEA complex Note: The Rag GTPase complex corresponds to Gtr1-Gtr2 GTPase complex ; GO:1990131. References: PMID:21454883, PMID:23974112 Sources: GOC:jh